cytoplasmic ubiquitin ligase complex [GO:0000153] (CC) Relationships: is a type of ubiquitin ligase complex [GO:0000151]; is part of cytoplasm [GO:0005737] Sources: GOC:mah Subtypes: ER ubiquitin ligase complex [GO:0000835], VCB complex [GO:0030891], cytoplasmic SCF ubiquitin ligase complex [GO:0043223] Definition: A ubiquitin ligase complex found in the cytoplasm.